1-acylglycerophosphoethanolamine O-acyltransferase activity [GO:0106262] (molecular function) Definition: Catalysis of the reaction: a 1-acyl-sn-glycero-3-phosphoethanolamine + an acyl-CoA = a 1,2-diacyl-sn-glycero-3-phosphoethanolamine + CoA. Relationships: is a type of O-acyltransferase activity [GO:0008374] References: PMID:18287005 Sources: RHEA:32995